positive regulation of chemotaxis [GO:0050921] (BP) Also known as: up regulation of chemotaxis, up-regulation of chemotaxis, upregulation of chemotaxis, activation of chemotaxis, stimulation of chemotaxis Sources: GOC:ai Relationships: is a type of positive regulation of response to external stimulus [GO:0032103]; is a type of positive regulation of locomotion [GO:0040017]; is_a regulation of chemotaxis [GO:0050920]; positively regulates chemotaxis [GO:0006935] Subtypes: positive regulation of leukocyte chemotaxis [GO:0002690], positive regulation of axon extension involved in axon guidance [GO:0048842], GO:0050924, positive regulation of positive chemotaxis [GO:0050927], GO:0071673, positive regulation of Schwann cell chemotaxis [GO:1904268], GO:1904554, positive regulation of cell chemotaxis to fibroblast growth factor [GO:1904849], positive regulation of endothelial cell chemotaxis to vascular endothelial growth factor [GO:1904859], positive regulation of fibroblast chemotaxis [GO:1905212], positive regulation of astrocyte chemotaxis [GO:2000464], positive regulation of endothelial cell chemotaxis [GO:2001028] Definition: Any process that activates or increases the frequency, rate or extent of the directed movement of a motile cell or organism in response to a specific chemical concentration gradient.